{
  "term_id": "GO:0019955",
  "gene_name": "Cytokine receptor common subunit gamma",
  "gene_symbol": "IL2RG",
  "term_label": "cytokine binding",
  "gene": "UniProtKB:P31785"
}